{
  "term_label": "homophilic cell-cell adhesion",
  "gene_name": "Hemicentin-2",
  "gene_symbol": "HMCN2",
  "gene": "UniProtKB:Q8NDA2",
  "term_id": "GO:0007156"
}